{
  "gene_symbol": "ZBTB17",
  "gene": "UniProtKB:Q13105",
  "term_label": "regulation of cytokine production",
  "gene_name": "Zinc finger and BTB domain-containing protein 17",
  "term_id": "GO:0001817"
}